{
  "gene_name": "Dynein axonemal assembly factor 8",
  "term_label": "Unknown biological process",
  "term_id": "UNKNOWN:0002",
  "gene": "UniProtKB:Q8IYS4",
  "gene_symbol": "DNAAF8"
}